{
  "gene": "UniProtKB:Q8TF47",
  "gene_name": "Zinc finger protein 90 homolog",
  "gene_symbol": "ZFP90",
  "term_id": "GO:0006357",
  "term_label": "regulation of transcription by RNA polymerase II"
}